{
  "gene": "UniProtKB:Q7Z6M4",
  "term_id": "GO:0061668",
  "term_label": "mitochondrial ribosome assembly",
  "gene_name": "Transcription termination factor 4, mitochondrial",
  "gene_symbol": "MTERF4"
}